{
  "gene": "UniProtKB:P17693",
  "term_id": "GO:0002476",
  "gene_symbol": "HLA-G",
  "term_label": "antigen processing and presentation of endogenous peptide antigen via MHC class Ib",
  "gene_name": "HLA class I histocompatibility antigen, alpha chain G"
}